cytokine receptor activity [GO:0004896] (molecular function) Definition: Combining with a cytokine and transmitting the signal from one side of the membrane to the other to initiate a change in cell activity. Also known as: IL receptor, interleukin receptor activity, hematopoietin/interferon-class (D200-domain) cytokine receptor activity Relationships: is a type of transmembrane signaling receptor activity [GO:0004888]; is a type of immune receptor activity [GO:0140375]; is part of cytokine-mediated signaling pathway [GO:0019221]; has part GO:0019955 Subtypes: interleukin-21 receptor activity [GO:0001532], GO:0002114, ciliary neurotrophic factor receptor activity [GO:0004897], erythropoietin receptor activity [GO:0004900], GO:0004901, granulocyte colony-stimulating factor receptor activity [GO:0004902], growth hormone receptor activity [GO:0004903], interferon receptor activity [GO:0004904], GO:0004908, interleukin-2 receptor activity [GO:0004911], interleukin-3 receptor activity [GO:0004912], interleukin-4 receptor activity [GO:0004913], GO:0004914, interleukin-6 receptor activity [GO:0004915], interleukin-7 receptor activity [GO:0004917], interleukin-9 receptor activity [GO:0004919], interleukin-10 receptor activity [GO:0004920], interleukin-11 receptor activity [GO:0004921], oncostatin-M receptor activity [GO:0004924], GO:0004925, chemokine receptor activity [GO:0004950], glial cell-derived neurotrophic factor receptor activity [GO:0016167], interleukin-13 receptor activity [GO:0016515], interleukin-12 receptor activity [GO:0016517], GO:0030368, leptin receptor activity [GO:0038021], thrombopoietin receptor activity [GO:0038164], interleukin-18 receptor activity [GO:0042008], interleukin-15 receptor activity [GO:0042010], interleukin-16 receptor activity [GO:0042012], interleukin-19 receptor activity [GO:0042014], interleukin-20 receptor activity [GO:0042016], interleukin-22 receptor activity [GO:0042018], interleukin-23 receptor activity [GO:0042020], interleukin-24 receptor activity [GO:0045506], interleukin-26 receptor activity [GO:0045508], high mobility group box 1 receptor activity [GO:0070380], interleukin-35 receptor activity [GO:0070747] Sources: GOC:add, GOC:mah